negative regulation of metanephric mesenchymal cell migration [GO:2000590] (biological process) Relationships: is_a negative regulation of cell migration [GO:0030336]; is_a negative regulation of metanephros development [GO:0072217]; is a type of regulation of metanephric mesenchymal cell migration [GO:2000589]; RO_0002212 metanephric mesenchymal cell migration [GO:0035789] Sources: GOC:obol Also known as: negative regulation of metanephric mesenchyme chemotaxis Definition: Any process that stops, prevents or reduces the frequency, rate or extent of metanephric mesenchymal cell migration.